negative regulation of podocyte apoptotic process [GO:1904634] (biological process) Definition: Any process that stops, prevents or reduces the frequency, rate or extent of glomerular visceral epithelial cell apoptotic process. References: PMID:23692924 Sources: GOC:TermGenie, GO_REF:0000058 Also known as: down regulation of glomerular podocyte apoptotic process, down regulation of glomerular visceral epithelial cell apoptotic process, down regulation of podocyte apoptotic process, down-regulation of glomerular podocyte apoptotic process, down-regulation of glomerular visceral epithelial cell apoptotic process, down-regulation of podocyte apoptotic process, downregulation of glomerular podocyte apoptotic process, downregulation of glomerular visceral epithelial cell apoptotic process, downregulation of podocyte apoptotic process, negative regulation of glomerular podocyte apoptotic process, negative regulation of glomerular visceral epithelial cell apoptotic process, negative regulation of podocyte apoptosis, down regulation of glomerular podocyte apoptosis, down regulation of glomerular visceral epithelial cell apoptosis, down regulation of podocyte apoptosis, down-regulation of glomerular podocyte apoptosis, down-regulation of glomerular visceral epithelial cell apoptosis, down-regulation of podocyte apoptosis, downregulation of glomerular podocyte apoptosis, downregulation of glomerular visceral epithelial cell apoptosis, downregulation of podocyte apoptosis, inhibition of glomerular podocyte apoptosis, inhibition of glomerular podocyte apoptotic process, inhibition of glomerular visceral epithelial cell apoptosis, inhibition of glomerular visceral epithelial cell apoptotic process, inhibition of podocyte apoptosis, inhibition of podocyte apoptotic process, negative regulation of glomerular podocyte apoptosis, negative regulation of glomerular visceral epithelial cell apoptosis Relationships: is a type of negative regulation of epithelial cell apoptotic process [GO:1904036]; is a type of regulation of podocyte apoptotic process [GO:1904633]; RO_0002212 GO:1903210